positive regulation of mast cell degranulation [GO:0043306] (BP) Relationships: is a type of positive regulation of leukocyte degranulation [GO:0043302]; is a type of regulation of mast cell degranulation [GO:0043304]; positively regulates mast cell degranulation [GO:0043303] Also known as: positive regulation of mast cell granule exocytosis, up regulation of mast cell degranulation, up-regulation of mast cell degranulation, upregulation of mast cell degranulation, activation of mast cell degranulation, stimulation of mast cell degranulation Definition: Any process that activates or increases the frequency, rate or extent of mast cell degranulation. Sources: ISBN:0781735149 Subtypes: positive regulation of histamine secretion by mast cell [GO:1903595]